{
  "term_label": "transmembrane signaling receptor activity",
  "gene_symbol": "ANTXRL",
  "term_id": "GO:0004888",
  "gene_name": "Anthrax toxin receptor-like",
  "gene": "UniProtKB:A6NF34"
}